apoptotic process involved in blood vessel morphogenesis [GO:1902262] (biological process) References: PMID:16163358 Sources: GOC:TermGenie, GOC:dph, GOC:mtg_apoptosis Relationships: is a type of apoptotic process involved in morphogenesis [GO:0060561]; is part of blood vessel morphogenesis [GO:0048514] Also known as: apoptotic cell death involved in patterning of blood vessels, apoptotic programmed cell death involved in patterning of blood vessels, programmed cell death by apoptosis involved in patterning of blood vessels, apoptosis involved in patterning of blood vessels, apoptotic program involved in patterning of blood vessels, type I programmed cell death involved in patterning of blood vessels, signaling (initiator) caspase activity involved in patterning of blood vessels Definition: Any apoptotic process that is involved in blood vessel morphogenesis.